{
  "term_label": "ubiquitin protein ligase activity",
  "term_id": "GO:0061630",
  "gene_name": "Putative tripartite motif-containing protein 49B",
  "gene": "UniProtKB:A6NDI0",
  "gene_symbol": "TRIM49B"
}